{
  "gene_symbol": "LRP10",
  "term_label": "plasma membrane",
  "gene": "UniProtKB:Q7Z4F1",
  "gene_name": "Low-density lipoprotein receptor-related protein 10",
  "term_id": "GO:0005886"
}